{
  "gene_name": "Zinc finger protein 575",
  "gene_symbol": "ZNF575",
  "gene": "UniProtKB:Q86XF7",
  "term_id": "UNKNOWN:0003",
  "term_label": "Unknown cellular component"
}